symbiont-mediated generation of symbiont replication vacuole [GO:0141213] (biological process) Definition: A process in which a symbiont alters or subverts vacuole organization in its host organism to form a protected environment in which it can replicate. The host is defined as the larger of the organisms involved in a symbiotic interaction. Relationships: is a type of symbiont-mediated perturbation of host vacuole organization [GO:0044075] References: PMID:21822290, PMID:23186105, PMID:30893609